{
  "gene_symbol": "SYAP1",
  "gene_name": "Synapse-associated protein 1",
  "term_id": "UNKNOWN:0001",
  "term_label": "Unknown molecular function",
  "gene": "UniProtKB:Q96A49"
}